{
  "term_id": "GO:0000922",
  "gene_symbol": "LATS2",
  "term_label": "spindle pole",
  "gene_name": "Serine_threonine-protein kinase LATS2",
  "gene": "UniProtKB:Q9NRM7"
}